positive regulation of plant-type hypersensitive response [GO:0034052] (biological process) Relationships: is a type of regulation of plant-type hypersensitive response [GO:0010363]; is a type of GO:0043068; is a type of positive regulation of innate immune response [GO:0045089]; positively regulates GO:0009626 Sources: GOC:pamgo_curators Definition: Any process that activates or increases the frequency, rate or extent of the hypersensitive response in a plant. Also known as: positive regulation of HR, positive regulation of plant hypersensitive response, up regulation of plant-type hypersensitive response, up-regulation of plant-type hypersensitive response, upregulation of plant-type hypersensitive response, activation of plant-type hypersensitive response, stimulation of plant-type hypersensitive response, positive regulation of HR-PCD